{
  "gene_symbol": "FKBPL",
  "gene": "UniProtKB:Q9UIM3",
  "term_label": "Unknown molecular function",
  "gene_name": "FK506-binding protein-like",
  "term_id": "UNKNOWN:0001"
}